{
  "term_label": "olfactory receptor activity",
  "gene": "UniProtKB:Q8NGK3",
  "gene_name": "Olfactory receptor 52K2",
  "gene_symbol": "OR52K2",
  "term_id": "GO:0004984"
}